{
  "gene": "UniProtKB:Q9UJ99",
  "gene_symbol": "CDH22",
  "gene_name": "Cadherin-22",
  "term_id": "GO:0008013",
  "term_label": "beta-catenin binding"
}